negative regulation of gene silencing by regulatory ncRNA [GO:0060967] (biological process) Subtypes: GO:0060906, GO:1900369 Definition: Any process that decreases the rate, frequency, or extent of gene silencing by RNA. Gene silencing by RNA is the process in which RNA molecules inactivate expression of target genes. Also known as: negative regulation of gene silencing by RNA, negative regulation of gene silencing by ncRNA Relationships: is a type of positive regulation of gene expression [GO:0010628]; is a type of negative regulation of biological process [GO:0048519]; is a type of regulation of gene silencing by regulatory ncRNA [GO:0060966]; negatively regulates GO:0031047 Sources: GOC:dph, GOC:tb